{
  "term_label": "Unknown biological process",
  "gene_symbol": "DDN",
  "gene": "UniProtKB:O94850",
  "gene_name": "Dendrin",
  "term_id": "UNKNOWN:0002"
}